{
  "gene_name": "Phospholipase A2",
  "term_label": "calcium-dependent phospholipase A2 activity",
  "gene": "UniProtKB:P04054",
  "term_id": "GO:0047498",
  "gene_symbol": "PLA2G1B"
}